{
  "gene_symbol": "TNFRSF10C",
  "term_id": "GO:0009986",
  "gene": "UniProtKB:O14798",
  "term_label": "cell surface",
  "gene_name": "Tumor necrosis factor receptor superfamily member 10C"
}